{
  "gene": "UniProtKB:Q8IY85",
  "term_label": "Unknown cellular component",
  "gene_symbol": "EFCAB13",
  "term_id": "UNKNOWN:0003",
  "gene_name": "EF-hand calcium-binding domain-containing protein 13"
}